{
  "term_label": "regulation of mitochondrion organization",
  "gene_name": "Polyamine-transporting ATPase 13A2",
  "gene_symbol": "ATP13A2",
  "term_id": "GO:0010821",
  "gene": "UniProtKB:Q9NQ11"
}